{
  "gene": "UniProtKB:Q9UBC9",
  "term_id": "UNKNOWN:0003",
  "term_label": "Unknown cellular component",
  "gene_name": "Small proline-rich protein 3",
  "gene_symbol": "SPRR3"
}